{
  "gene_name": "Damage-control phosphatase ARMT1",
  "gene_symbol": "ARMT1",
  "term_label": "phosphatase activity",
  "gene": "UniProtKB:Q9H993",
  "term_id": "GO:0016791"
}